lymphocyte activation [GO:0046649] (biological process) Regulation: regulated by regulation of lymphocyte activation [GO:0051249]; negatively regulated by negative regulation of lymphocyte activation [GO:0051250]; positively regulated by GO:0051251 Relationships: is a type of GO:0045321 Definition: A change in morphology and behavior of a lymphocyte resulting from exposure to a specific antigen, mitogen, cytokine, chemokine, cellular ligand, or soluble factor. Subtypes: lymphocyte activation involved in immune response [GO:0002285], lymphocyte differentiation [GO:0030098], natural killer cell activation [GO:0030101], T cell activation [GO:0042110], GO:0042113, GO:0046651 Sources: GOC:mgi_curators, ISBN:0781735149